chaperone-mediated autophagy [GO:0061684] (biological process) Definition: The autophagy process which begins when chaperones and co-chaperones recognize a target motif and unfold the substrate protein. The proteins are then transported to the lysosome where they are degraded. References: PMID:22743996, PMID:23434281 Sources: GOC:PARL, GOC:pad Also known as: CASA, CMA, chaperone-assisted selective autophagy Relationships: is a type of GO:0006914; is a type of protein catabolic process [GO:0030163]; BFO_0000051 signaling receptor binding [GO:0005102]; has part GO:0051087; has part protein carrier chaperone [GO:0140597] Regulation: regulated by GO:1904714; negatively regulated by negative regulation of chaperone-mediated autophagy [GO:1904715]; positively regulated by GO:1904716